anatomical structure homeostasis [GO:0060249] (BP) Definition: A homeostatic process involved in the maintenance of an internal steady state within a defined anatomical structure of an organism, including control of cellular proliferation and death and control of metabolic function. An anatomical structure is any biological entity that occupies space and is distinguished from its surroundings. Anatomical structures can be macroscopic such as a carpel, or microscopic such as an acrosome. Sources: GOC:dph Also known as: anatomical structure maintenance Relationships: is a type of multicellular organismal-level homeostasis [GO:0048871] Subtypes: tissue homeostasis [GO:0001894], germ-line stem-cell niche homeostasis [GO:0060250]